{
  "gene_name": "Krueppel-like factor 4",
  "term_label": "regulation of transcription by RNA polymerase II",
  "gene": "UniProtKB:O43474",
  "term_id": "GO:0006357",
  "gene_symbol": "KLF4"
}